protein secretion by the type II secretion system [GO:0015628] (BP) Also known as: protein secretion by the T2S, protein secretion by the T2SS, protein secretion by the type II protein secretion system, type II protein secretion system, protein secretion by the general secretion pathway, protein secretion by the general secretory pathway Note: Note that this term represents an activity and not a cellular structure. Consider also annotating to the cellular component term 'type II protein secretion system complex ; GO:0015627'. This process refers specifically to secretion across the outer membrane. For components of the Sec and Tat pathways, consider annotating to 'protein transport by the Sec complex ; GO:0043952' and 'protein transport by the Tat complex ; GO:0043953'. Note that this term is used for annotation of proteins that compose the secretion complex but not the proteins being secreted. Definition: The process in which proteins are secreted across the outer membrane of Gram-negative bacteria by the type II secretion system. Proteins using this pathway are first translocated across the cytoplasmic membrane via the Sec or Tat pathways. Relationships: is a type of protein secretion [GO:0009306]; is a type of protein transport across the cell outer membrane [GO:0098776] Sources: GOC:pamgo_curators